{
  "gene_symbol": "RIC3",
  "gene": "UniProtKB:Q7Z5B4",
  "term_label": "neuronal cell body",
  "gene_name": "Protein RIC-3",
  "term_id": "GO:0043025"
}